negative regulation of nucleotide-binding oligomerization domain containing 2 signaling pathway [GO:0070433] (biological process) Definition: Any process that stops, prevents, or reduces the frequency, rate, or extent of the nucleotide-binding oligomerization domain containing 2 (NOD2) pathway. Also known as: negative regulation of NOD2 signaling pathway, negative regulation of nucleotide-binding oligomerization domain containing 2 signalling pathway Relationships: is a type of negative regulation of nucleotide-binding domain, leucine rich repeat containing receptor signaling pathway [GO:0070425]; is a type of GO:0070432; negatively regulates nucleotide-binding oligomerization domain containing 2 signaling pathway [GO:0070431] Sources: GOC:add